secondary active transmembrane transporter activity [GO:0015291] (molecular function) References: PMID:10839820 Sources: GOC:mtg_transport, ISBN:0198506732, ISBN:0815340729 Also known as: active transporter, coupled carrier, electrochemical potential-driven transporter activity, porter activity, porters, secondary carrier-type facilitators, energizer of outer membrane receptor-mediated transport activity, heavy metal ion porter activity, ion-gradient-driven energizer activity, multidrug endosomal transmembrane transporter activity, nitrite/nitrate porter activity, galactose/glucose (methylgalactoside) porter activity Definition: Enables the transfer of a solute from one side of a membrane to the other, up its concentration gradient. The transporter binds the solute and undergoes a series of conformational changes. Transport works equally well in either direction and is driven by a chemiosmotic source of energy, not direct ATP coupling. Secondary active transporters include symporters and antiporters. Subtypes: neutral L-amino acid secondary active transmembrane transporter activity [GO:0005294], phosphate transmembrane transporter activity [GO:0005315], tricarboxylate secondary active transmembrane transporter activity [GO:0005371], proton-dependent oligopeptide secondary active transmembrane transporter activity [GO:0005427], secondary active sulfate transmembrane transporter activity [GO:0008271], GO:0008490, GO:0009977, nucleoside transmembrane transporter activity, against a concentration gradient [GO:0010174], GO:0015292, symporter activity [GO:0015293], antiporter activity [GO:0015297], GO:0015349, secondary active monocarboxylate transmembrane transporter activity [GO:0015355], high-affinity secondary active nitrite transmembrane transporter activity [GO:0015513], nitrite efflux transmembrane transporter activity [GO:0015514], secondary active cyanate transmembrane transporter activity [GO:0015541], secondary active p-aminobenzoyl-glutamate transmembrane transporter activity [GO:0015558], antimonite secondary active transmembrane transporter activity [GO:0042960] Relationships: is a type of GO:0022804